{
  "gene_name": "Type-1 angiotensin II receptor",
  "term_label": "positive regulation of cytosolic calcium ion concentration",
  "term_id": "GO:0007204",
  "gene_symbol": "AGTR1",
  "gene": "UniProtKB:P30556"
}